{
  "term_id": "GO:0019287",
  "gene_symbol": "PMVK",
  "term_label": "isopentenyl diphosphate biosynthetic process, mevalonate pathway",
  "gene_name": "Phosphomevalonate kinase",
  "gene": "UniProtKB:Q15126"
}